{
  "gene_symbol": "SLC24A4",
  "term_label": "calcium channel activity",
  "gene": "UniProtKB:Q8NFF2",
  "gene_name": "Sodium_potassium_calcium exchanger 4",
  "term_id": "GO:0005262"
}